{
  "term_id": "GO:0016567",
  "term_label": "protein ubiquitination",
  "gene_symbol": "CBLL2",
  "gene": "UniProtKB:Q8N7E2",
  "gene_name": "E3 ubiquitin-protein ligase CBLL2"
}